apical lamina of hyaline layer [GO:0032579] (cellular component) Definition: A fibrous network that is part of the hyalin layer extracellular matrix. The apical lamina is thought to be principally composed of the glycoproteins fibropellins. This matrix has been found in echinoderms. Relationships: is a type of cellular anatomical structure [GO:0110165]; is part of GO:0033166 References: PMID:2060714, PMID:7608987, PMID:9638331 Sources: GOC:ecd